{
  "term_label": "immunoglobulin complex",
  "gene_symbol": "IGKV1D-8",
  "term_id": "GO:0019814",
  "gene": "UniProtKB:A0A087WSZ0",
  "gene_name": "Immunoglobulin kappa variable 1D-8"
}